pyloric sphincter smooth muscle contraction [GO:0120067] (biological process) Definition: A process in which force is generated within gastric smooth muscle tissue, resulting in a change in muscle geometry. This process occurs in the narrowest part of the pylorus that separates the stomach from the duodenum. References: PMID:15890336 Sources: GOC:sl Relationships: is a type of GO:0120064